{
  "gene": "UniProtKB:Q9UKB1",
  "term_label": "germ cell development",
  "gene_name": "F-box_WD repeat-containing protein 11",
  "term_id": "GO:0007281",
  "gene_symbol": "FBXW11"
}